{
  "gene_name": "Procollagen-lysine,2-oxoglutarate 5-dioxygenase 1",
  "term_id": "GO:0005783",
  "term_label": "endoplasmic reticulum",
  "gene": "UniProtKB:Q02809",
  "gene_symbol": "PLOD1"
}